{
  "gene_symbol": "NBPF19",
  "gene_name": "Neuroblastoma breakpoint family member 19",
  "term_label": "Unknown cellular component",
  "term_id": "UNKNOWN:0003",
  "gene": "UniProtKB:A0A087WUL8"
}